{
  "term_id": "UNKNOWN:0001",
  "gene_name": "COP9 signalosome complex subunit 6",
  "term_label": "Unknown molecular function",
  "gene": "UniProtKB:Q7L5N1",
  "gene_symbol": "COPS6"
}